negative regulation of cell migration [GO:0030336] (biological process) Also known as: down regulation of cell migration, down-regulation of cell migration, downregulation of cell migration, inhibition of cell migration Relationships: is a type of regulation of cell migration [GO:0030334]; is_a GO:2000146; negatively regulates cell migration [GO:0016477] Subtypes: negative regulation of leukocyte migration [GO:0002686], GO:0010596, negative regulation of epithelial cell migration [GO:0010633], negative regulation of fibroblast migration [GO:0010764], negative regulation of smooth muscle cell migration [GO:0014912], neuromast deposition [GO:0048885], negative regulation of neuroblast migration [GO:0061855], negative regulation of myotube cell migration [GO:0110125], negative regulation of chemokine activity [GO:1900137], GO:1901164, negative regulation of distal tip cell migration [GO:1903355], negative regulation of wound healing, spreading of epidermal cells [GO:1903690], negative regulation of glial cell migration [GO:1903976], negative regulation of substrate-dependent cell migration, cell attachment to substrate [GO:1904236], negative regulation of cell chemotaxis to fibroblast growth factor [GO:1904848], GO:1904858, negative regulation of fibroblast chemotaxis [GO:1905211], negative regulation of cardiac neural crest cell migration involved in outflow tract morphogenesis [GO:1905311], negative regulation of mesenchymal stem cell migration [GO:1905321], negative regulation of hematopoietic stem cell migration [GO:2000472], GO:2000590, negative regulation of neuron migration [GO:2001223], negative regulation of muscle cell chemotaxis toward tendon cell [GO:2001282] Definition: Any process that stops, prevents, or reduces the frequency, rate or extent of cell migration. Sources: GOC:go_curators